regulation of lamellipodium morphogenesis [GO:2000392] (biological process) Definition: Any process that modulates the frequency, rate or extent of lamellipodium morphogenesis. Relationships: is a type of regulation of cell morphogenesis [GO:0022604]; is a type of GO:1902743; regulates GO:0072673 Sources: GOC:mah Also known as: regulation of lamellipodium organization Subtypes: GO:2000393, positive regulation of lamellipodium morphogenesis [GO:2000394]